{
  "term_id": "GO:0070330",
  "gene": "UniProtKB:P11511",
  "term_label": "aromatase activity",
  "gene_symbol": "CYP19A1",
  "gene_name": "Aromatase"
}